{
  "term_label": "double-stranded DNA binding",
  "gene": "UniProtKB:P41218",
  "gene_name": "Myeloid cell nuclear differentiation antigen",
  "gene_symbol": "MNDA",
  "term_id": "GO:0003690"
}